negative regulation of blood circulation [GO:1903523] (biological process) Subtypes: GO:0045822, negative regulation of cerebral blood circulation [GO:0120278], negative regulation of gastric mucosal blood circulation [GO:1904345] Definition: Any process that stops, prevents or reduces the frequency, rate or extent of blood circulation. Relationships: is a type of negative regulation of multicellular organismal process [GO:0051241]; is_a regulation of blood circulation [GO:1903522]; negatively regulates blood circulation [GO:0008015] Also known as: down regulation of blood circulation, down-regulation of blood circulation, downregulation of blood circulation, inhibition of blood circulation, down regulation of hemolymph circulation, down-regulation of hemolymph circulation, downregulation of hemolymph circulation, inhibition of hemolymph circulation, negative regulation of hemolymph circulation References: PMID:10659969 Sources: GOC:TermGenie, GOC:mr, GO_REF:0000058